basophil differentiation [GO:0030221] (biological process) Regulation: regulated by regulation of basophil differentiation [GO:0045640]; negatively regulated by negative regulation of basophil differentiation [GO:0045641]; positively regulated by positive regulation of basophil differentiation [GO:0045642] Sources: GOC:jid, GOC:mah Relationships: is a type of granulocyte differentiation [GO:0030851] Definition: The process in which a relatively unspecialized myeloid precursor cell acquires specialized features of a basophil cell. Also known as: basophil cell differentiation